IgM immunoglobulin complex, circulating [GO:0071754] (cellular component) Note: Note that an IgM immunoglobulin complex has the function of antigen binding if a suitable antigen is available. Definition: A polymer of five or six IgM core units each composed of two identical immunoglobulin heavy chains of the IgM isotype and two identical immunoglobulin light chains, held together by disulfide bonds; the individual IgM core units are held together via disulfide bonds with a single J chain polypeptide acting as a bridge between two of the polymeric units. Circulating IgM is present in the extracellular space, in mucosal areas or other tissues, or in the blood or lymph. References: PMID:20176268 Sources: GOC:add, ISBN:0781765196 Relationships: is a type of immunoglobulin complex, circulating [GO:0042571]; is a type of IgM immunoglobulin complex [GO:0071753] Subtypes: pentameric IgM immunoglobulin complex [GO:0071756], hexameric IgM immunoglobulin complex [GO:0071757] Also known as: IgM antibody